{
  "gene": "UniProtKB:O00358",
  "term_label": "RNA polymerase II cis-regulatory region sequence-specific DNA binding",
  "term_id": "GO:0000978",
  "gene_symbol": "FOXE1",
  "gene_name": "Forkhead box protein E1"
}